{
  "gene_name": "Charged multivesicular body protein 4a",
  "gene_symbol": "CHMP4A",
  "term_id": "GO:0006900",
  "term_label": "vesicle budding from membrane",
  "gene": "UniProtKB:Q9BY43"
}